{
  "gene_symbol": "ITGB1",
  "gene": "UniProtKB:P05556",
  "term_label": "integrin-mediated signaling pathway",
  "term_id": "GO:0007229",
  "gene_name": "Integrin beta-1"
}